regulation of macropinocytosis [GO:1905301] (biological process) Definition: Any process that modulates the frequency, rate or extent of macropinocytosis. Subtypes: negative regulation of macropinocytosis [GO:1905302], positive regulation of macropinocytosis [GO:1905303] References: PMID:18691641 Sources: GOC:PARL, GOC:TermGenie, GOC:pad, GO_REF:0000058 Also known as: regulation of clathrin-independent pinocytosis Relationships: is a type of regulation of pinocytosis [GO:0048548]; RO_0002211 macropinocytosis [GO:0044351]